actin cap [GO:0030478] (cellular component) Definition: Polarized accumulation of cytoskeletal proteins (including F-actin) and regulatory proteins in a cell. An example of this is the actin cap found in Saccharomyces cerevisiae. References: PMID:21494665 Sources: GOC:mah Relationships: is a type of cellular anatomical structure [GO:0110165]; is part of cortical actin cytoskeleton [GO:0030864]